{
  "gene_name": "cAMP-specific 3',5'-cyclic phosphodiesterase 7B",
  "term_label": "Unknown cellular component",
  "term_id": "UNKNOWN:0003",
  "gene": "UniProtKB:Q9NP56",
  "gene_symbol": "PDE7B"
}